Lewy body core [GO:1990037] (cellular component) Relationships: is a type of cellular anatomical structure [GO:0110165]; is part of GO:0097413 Sources: NIF_Subcellular:sao6587439252 Definition: The center portion of a Lewy body. In Parkinson's disease, it contains a matted meshwork of filaments.